{
  "gene_name": "Mitochondrial import inner membrane translocase subunit Tim23",
  "gene_symbol": "TIMM23",
  "gene": "UniProtKB:O14925",
  "term_id": "GO:0005744",
  "term_label": "TIM23 mitochondrial import inner membrane translocase complex"
}